{
  "gene": "UniProtKB:Q9Y6X1",
  "gene_name": "Stress-associated endoplasmic reticulum protein 1",
  "gene_symbol": "SERP1",
  "term_label": "Unknown molecular function",
  "term_id": "UNKNOWN:0001"
}